positive regulation of isotype switching to IgA isotypes [GO:0048298] (biological process) Relationships: is a type of GO:0045830; is a type of regulation of isotype switching to IgA isotypes [GO:0048296]; positively regulates isotype switching to IgA isotypes [GO:0048290] Definition: Any process that activates or increases the frequency, rate or extent of isotype switching to IgA isotypes. Also known as: positive regulation of class switch recombination to IgA isotypes, positive regulation of class switching to IgA isotypes, positive regulation of isotype switch recombination to IgA isotypes, up regulation of isotype switching to IgA isotypes, up-regulation of isotype switching to IgA isotypes, upregulation of isotype switching to IgA isotypes, activation of isotype switching to IgA isotypes, stimulation of isotype switching to IgA isotypes Sources: GOC:jid